{
  "gene_symbol": "ZNF114",
  "term_id": "GO:0000981",
  "gene": "UniProtKB:Q8NC26",
  "term_label": "DNA-binding transcription factor activity, RNA polymerase II-specific",
  "gene_name": "Zinc finger protein 114"
}